{
  "term_label": "fibroblast growth factor receptor signaling pathway",
  "gene": "UniProtKB:Q9NSA1",
  "term_id": "GO:0008543",
  "gene_symbol": "FGF21",
  "gene_name": "Fibroblast growth factor 21"
}